{
  "gene_name": "Zinc finger C4H2 domain-containing protein",
  "term_id": "GO:0045666",
  "gene_symbol": "ZC4H2",
  "term_label": "positive regulation of neuron differentiation",
  "gene": "UniProtKB:Q9NQZ6"
}